{
  "gene_name": "Coiled-coil domain-containing protein 134",
  "gene": "UniProtKB:Q9H6E4",
  "gene_symbol": "CCDC134",
  "term_label": "protein-macromolecule adaptor activity",
  "term_id": "GO:0030674"
}